host cell peroxisome [GO:0120149] (cellular component) Also known as: host peroxisome Definition: A small host cell organelle enclosed by a single membrane, and found in most eukaryotic cells. Contains peroxidases and other enzymes involved in a variety of metabolic processes including free radical detoxification, lipid catabolism and biosynthesis, and hydrogen peroxide metabolism. Relationships: is a type of host intracellular membrane-bounded organelle [GO:0033648]; is a type of host cell cytoplasm part [GO:0033655] References: PMID:9302272